{
  "gene_name": "Solute carrier family 66 member 2",
  "term_id": "GO:0042147",
  "gene_symbol": "SLC66A2",
  "term_label": "retrograde transport, endosome to Golgi",
  "gene": "UniProtKB:Q8N2U9"
}